{
  "term_id": "GO:0005886",
  "gene_symbol": "NEO1",
  "gene": "UniProtKB:Q92859",
  "term_label": "plasma membrane",
  "gene_name": "Neogenin"
}